positive regulation of phosphatidylserine exposure on apoptotic cell surface [GO:1905782] (biological process) Relationships: is a type of GO:0061092; is a type of regulation of phosphatidylserine exposure on apoptotic cell surface [GO:1905780]; positively regulates phosphatidylserine exposure on apoptotic cell surface [GO:0070782] Also known as: positive regulation of externalization of phosphatidylserine, up regulation of externalization of phosphatidylserine, up regulation of phosphatidylserine exposure on apoptotic cell surface, up-regulation of externalization of phosphatidylserine, up-regulation of phosphatidylserine exposure on apoptotic cell surface, upregulation of externalization of phosphatidylserine, upregulation of phosphatidylserine exposure on apoptotic cell surface, activation of externalization of phosphatidylserine, activation of phosphatidylserine exposure on apoptotic cell surface References: PMID:17401362 Sources: GOC:TermGenie, GOC:kmv, GO_REF:0000058 Definition: Any process that activates or increases the frequency, rate or extent of phosphatidylserine exposure on apoptotic cell surface.